U2-type prespliceosome assembly [GO:1903241] (biological process) Definition: The aggregation, arrangement and bonding together of a set of components to form an U2-type prespliceosome. References: PMID:12374752 Sources: GOC:TermGenie, GO_REF:0000079 Also known as: U2-type prespliceosome formation, major prespliceosome assembly, major prespliceosome formation, GT-AG prespliceosome assembly, GT-AG prespliceosome formation, mammalian U2-type spliceosomal complex A assembly, mammalian U2-type spliceosomal complex A formation, yeast U2-type spliceosomal complex B assembly, yeast U2-type spliceosomal complex B formation Relationships: is a type of GO:0000245